{
  "gene_name": "Ubiquitin-conjugating enzyme E2 D1",
  "gene_symbol": "UBE2D1",
  "term_label": "ubiquitin conjugating enzyme activity",
  "gene": "UniProtKB:P51668",
  "term_id": "GO:0061631"
}